{
  "gene": "UniProtKB:Q2VIQ3",
  "term_label": "mitotic spindle organization",
  "gene_symbol": "KIF4B",
  "term_id": "GO:0007052",
  "gene_name": "Chromosome-associated kinesin KIF4B"
}